{
  "gene_name": "Histone H2A type 1-A",
  "gene": "UniProtKB:Q96QV6",
  "term_id": "GO:0031507",
  "term_label": "heterochromatin formation",
  "gene_symbol": "H2AC1"
}